protein localization to mitotic actomyosin contractile ring [GO:1904498] (biological process) References: PMID:25688133 Sources: GOC:TermGenie, GO_REF:0000060 Definition: Any protein localization to actomyosin contractile ring that is involved in mitotic cytokinesis. Also known as: protein localisation to actomyosin contractile ring involved in cytokinesis after mitosis, protein localisation to actomyosin contractile ring involved in mitotic cytokinesis, protein localization to actomyosin contractile ring involved in cytokinesis after mitosis, protein localization to actomyosin contractile ring involved in mitotic cytokinesis, protein localization to actomyosin contractile ring during mitotic cytokinesis Relationships: is_a GO:1990179; BFO_0000050 mitotic cytokinesis [GO:0000281]